negative regulation of fat cell differentiation [GO:0045599] (biological process) Definition: Any process that stops, prevents, or reduces the frequency, rate or extent of adipocyte differentiation. Sources: GOC:go_curators Also known as: down regulation of fat cell differentiation, down-regulation of fat cell differentiation, downregulation of fat cell differentiation, negative regulation of adipocyte cell differentiation, negative regulation of adipocyte differentiation, inhibition of fat cell differentiation Subtypes: negative regulation of white fat cell differentiation [GO:0160275], negative regulation of beige fat cell differentiation [GO:0160276], negative regulation of brown fat cell differentiation [GO:1903444] Relationships: is a type of negative regulation of cell differentiation [GO:0045596]; is a type of regulation of fat cell differentiation [GO:0045598]; negatively regulates fat cell differentiation [GO:0045444]